{
  "gene_name": "Ras-related protein Rab-31",
  "gene": "UniProtKB:Q13636",
  "term_id": "GO:0032588",
  "gene_symbol": "RAB31",
  "term_label": "trans-Golgi network membrane"
}